{
  "gene_symbol": "SPIB",
  "term_label": "regulation of transcription by RNA polymerase II",
  "gene_name": "Transcription factor Spi-B",
  "gene": "UniProtKB:Q01892",
  "term_id": "GO:0006357"
}